{
  "term_label": "Unknown biological process",
  "gene": "UniProtKB:Q14129",
  "gene_symbol": "DGCR6",
  "term_id": "UNKNOWN:0002",
  "gene_name": "Protein DGCR6"
}